{
  "term_id": "GO:0045202",
  "gene_name": "Microtubule-associated protein 1S",
  "gene": "UniProtKB:Q66K74",
  "term_label": "synapse",
  "gene_symbol": "MAP1S"
}